{
  "term_label": "neuron projection",
  "gene_symbol": "PICK1",
  "gene": "UniProtKB:Q9NRD5",
  "gene_name": "PRKCA-binding protein",
  "term_id": "GO:0043005"
}